{
  "gene_symbol": "GSTA2",
  "term_label": "xenobiotic metabolic process",
  "gene_name": "Glutathione S-transferase A2",
  "term_id": "GO:0006805",
  "gene": "UniProtKB:P09210"
}